{
  "gene_symbol": "LIMS3",
  "term_label": "Unknown biological process",
  "term_id": "UNKNOWN:0002",
  "gene": "UniProtKB:P0CW19",
  "gene_name": "LIM and senescent cell antigen-like-containing domain protein 3"
}